{
  "term_label": "DNA-binding transcription factor activity, RNA polymerase II-specific",
  "term_id": "GO:0000981",
  "gene_name": "T-cell leukemia homeobox protein 2",
  "gene_symbol": "TLX2",
  "gene": "UniProtKB:O43763"
}